{
  "term_id": "UNKNOWN:0001",
  "gene": "UniProtKB:A6NCF5",
  "term_label": "Unknown molecular function",
  "gene_name": "Kelch-like protein 33",
  "gene_symbol": "KLHL33"
}